L-histidine N(alpha)-methyltransferase activity [GO:0052706] (molecular function) Definition: Catalysis of the reaction: L-histidine + 3 S-adenosyl-L-methionine <=> 3 H(+) + hercynine + 3 S-adenosyl-L-homocysteine. This reaction is the addition of three methyl groups to L-histidine to form N-alpha,N-alpha,N-alpha-trimethyl-L-histidine (also known as hercynine). Also known as: S-adenosyl-L-methionine:L-histidine Nalpha-methyltransferase activity, S-adenosyl-L-methionine:L-histidine alpha-N-methyltransferase activity, histidine N-methyltransferase activity, histidine methyltransferase activity, histidine-alpha-N-methyltransferase activity Sources: RHEA:38471 Relationships: is a type of S-adenosylmethionine-dependent methyltransferase activity [GO:0008757]